{
  "gene_name": "UDP-N-acetylglucosamine transporter",
  "term_id": "GO:0055085",
  "gene": "UniProtKB:Q9Y2D2",
  "gene_symbol": "SLC35A3",
  "term_label": "transmembrane transport"
}